{
  "term_label": "Unknown molecular function",
  "gene_name": "Glutamate-rich protein 5",
  "gene_symbol": "ERICH5",
  "gene": "UniProtKB:Q6P6B1",
  "term_id": "UNKNOWN:0001"
}